{
  "gene_name": "Rho GTPase-activating protein 44",
  "gene": "UniProtKB:Q17R89",
  "term_id": "GO:0005886",
  "term_label": "plasma membrane",
  "gene_symbol": "ARHGAP44"
}